{
  "gene": "UniProtKB:P00167",
  "term_id": "UNKNOWN:0002",
  "gene_name": "Cytochrome b5",
  "gene_symbol": "CYB5A",
  "term_label": "Unknown biological process"
}